{
  "gene_symbol": "GNL1",
  "gene_name": "Guanine nucleotide-binding protein-like 1",
  "gene": "UniProtKB:P36915",
  "term_label": "GTPase activity",
  "term_id": "GO:0003924"
}